tubulin-glutamic acid ligase activity [GO:0070740] (molecular function) Definition: Catalysis of the posttranslational transfer of one or more glutamate residues to the gamma-carboxyl group(s) of one or more specific glutamate residues on a tubulin molecule. References: PMID:19524510 Sources: GOC:mah Relationships: is a type of protein-glutamic acid ligase activity [GO:0070739] Also known as: tubulin glutamylase activity, tubulin-glutamate ligase activity